{
  "term_label": "semaphorin receptor binding",
  "gene_name": "Semaphorin-3F",
  "gene_symbol": "SEMA3F",
  "gene": "UniProtKB:Q13275",
  "term_id": "GO:0030215"
}